{
  "gene_symbol": "GRIN1",
  "term_id": "GO:0045202",
  "gene": "UniProtKB:Q05586",
  "term_label": "synapse",
  "gene_name": "Glutamate receptor ionotropic, NMDA 1"
}